{
  "gene_symbol": "SEH1L",
  "gene": "UniProtKB:Q96EE3",
  "gene_name": "Nucleoporin SEH1",
  "term_label": "cellular response to amino acid starvation",
  "term_id": "GO:0034198"
}